proton-transporting ATPase activity, rotational mechanism [GO:0046961] (molecular function) Relationships: is a type of GO:0015078; is_a ATPase-coupled monoatomic cation transmembrane transporter activity [GO:0019829]; is a type of ATPase activity, coupled to transmembrane movement of ions, rotational mechanism [GO:0044769] Also known as: hydrogen ion transporting ATPase activity, rotational mechanism, ATP phosphohydrolase (H+-transporting) activity, ATP synthase activity, F(0)F(1)-ATPase activity, F(1)-ATPase activity, F(o)F(1)-ATPase activity, F0F1-ATPase, F1-ATPase, FoF1-ATPase, H+-transporting ATP synthase activity, H+-transporting ATPase activity, chloroplast ATPase activity, hydrogen ion translocating A-type ATPase activity, hydrogen ion translocating F-type ATPase activity, hydrogen ion translocating V-type ATPase activity, hydrogen ion transporting two-sector ATPase activity, mitochondrial ATPase activity Definition: Enables the transfer of protons from one side of a membrane to the other by a rotational mechanism according to the reaction: ATP + H2O + 4 H+(in) => ADP + phosphate + 5 H+(out). Sources: RHEA:57721